{
  "gene": "UniProtKB:Q96LR5",
  "gene_name": "Ubiquitin-conjugating enzyme E2 E2",
  "gene_symbol": "UBE2E2",
  "term_label": "protein K48-linked ubiquitination",
  "term_id": "GO:0070936"
}